{
  "gene": "UniProtKB:Q07065",
  "term_id": "GO:0005791",
  "gene_symbol": "CKAP4",
  "gene_name": "Cytoskeleton-associated protein 4",
  "term_label": "rough endoplasmic reticulum"
}